{
  "gene_name": "Beta,beta-carotene 15,15'-dioxygenase",
  "term_id": "UNKNOWN:0003",
  "term_label": "Unknown cellular component",
  "gene": "UniProtKB:Q9HAY6",
  "gene_symbol": "BCO1"
}